{
  "term_label": "DNA replication",
  "term_id": "GO:0006260",
  "gene_name": "ATP-dependent DNA helicase Q1",
  "gene": "UniProtKB:P46063",
  "gene_symbol": "RECQL"
}